{
  "term_label": "extracellular space",
  "gene_symbol": "TGFA",
  "gene_name": "Protransforming growth factor alpha",
  "term_id": "GO:0005615",
  "gene": "UniProtKB:P01135"
}